{
  "gene_name": "Lysine-specific demethylase 5D",
  "term_label": "nucleus",
  "term_id": "GO:0005634",
  "gene": "UniProtKB:Q9BY66",
  "gene_symbol": "KDM5D"
}